{
  "gene": "UniProtKB:Q6PCB7",
  "term_id": "GO:0005789",
  "gene_symbol": "SLC27A1",
  "gene_name": "Long-chain fatty acid transport protein 1",
  "term_label": "endoplasmic reticulum membrane"
}